{
  "gene_symbol": "VCAM1",
  "gene": "UniProtKB:P19320",
  "term_label": "plasma membrane",
  "gene_name": "Vascular cell adhesion protein 1",
  "term_id": "GO:0005886"
}